{
  "term_id": "GO:0004984",
  "gene_symbol": "OR6P1",
  "gene": "UniProtKB:Q8NGX9",
  "term_label": "olfactory receptor activity",
  "gene_name": "Olfactory receptor 6P1"
}